{
  "gene": "UniProtKB:Q8NFT8",
  "term_id": "GO:0005112",
  "gene_name": "Delta and Notch-like epidermal growth factor-related receptor",
  "term_label": "Notch binding",
  "gene_symbol": "DNER"
}